trimethylsulfonium-tetrahydrofolate N-methyltransferase activity [GO:0047147] (molecular function) Sources: EC:2.1.1.19, RHEA:13693 Definition: Catalysis of the reaction: (6S)-5,6,7,8-tetrahydrofolate + trimethylsulfonium = (6S)-5-methyl-5,6,7,8-tetrahydrofolate + dimethyl sulfide + H+. Relationships: is a type of N-methyltransferase activity [GO:0008170] Also known as: trimethylsulphonium-tetrahydrofolate N-methyltransferase activity, trimethylsulfonium-tetrahydrofolate methyltransferase activity, trimethylsulfonium:tetrahydrofolate N-methyltransferase activity